IgG receptor activity [GO:0019770] (molecular function) Definition: Combining with an immunoglobulin of an IgG isotype via the Fc region, and transmitting the signal from one side of the membrane to the other to initiate a change in cell activity. Sources: GOC:add, GOC:signaling, ISBN:0781735149 Subtypes: high-affinity IgG receptor activity [GO:0019771], low-affinity IgG receptor activity [GO:0019772] Relationships: is a type of immunoglobulin receptor activity [GO:0019763]; is part of Fc-gamma receptor signaling pathway [GO:0038094]; has part GO:0019864